{
  "term_label": "actin filament organization",
  "term_id": "GO:0007015",
  "gene_name": "Engulfment and cell motility protein 1",
  "gene": "UniProtKB:Q92556",
  "gene_symbol": "ELMO1"
}